{
  "term_id": "GO:0019901",
  "gene": "UniProtKB:Q12959",
  "gene_symbol": "DLG1",
  "term_label": "protein kinase binding",
  "gene_name": "Disks large homolog 1"
}